carboxylic acid binding [GO:0031406] (molecular function) Definition: Binding to a carboxylic acid, an organic acid containing one or more carboxyl (COOH) groups or anions (COO-). Subtypes: GO:0005542, gibberellin binding [GO:0010331], glycine binding [GO:0016594], glutamate binding [GO:0016595], L-ascorbic acid binding [GO:0031418], monocarboxylic acid binding [GO:0033293], sialic acid binding [GO:0033691], arginine binding [GO:0034618], phthalate binding [GO:0035273], flurbiprofen binding [GO:0035923], 3-sulfino-L-alanine binding [GO:0036127], GO:0046904, GO:0050542, methotrexate binding [GO:0051870], dihydrofolic acid binding [GO:0051871], aspartate binding [GO:0070335], glutamine binding [GO:0070406], L-leucine binding [GO:0070728], serine binding [GO:0070905], GO:0070967, pyrroloquinoline quinone binding [GO:0070968], L-DOPA binding [GO:0072544], L-tyrosine binding [GO:0072545], tryptophan binding [GO:0120284], proline binding [GO:1901973], (25S)-Delta(4)-dafachronate binding [GO:1902051], GO:1902052, GO:1902485, GO:1904399, GO:1905573, ganglioside GM2 binding [GO:1905574], ganglioside GT1b binding [GO:1905576], ganglioside GP1c binding [GO:1905577] Sources: GOC:mah, ISBN:0198506732 Relationships: is a type of anion binding [GO:0043168]; is a type of organic acid binding [GO:0043177]